spore germination [GO:0009847] (biological process) Definition: The physiological and developmental changes that occur in a spore following release from dormancy up to the earliest signs of growth (e.g. emergence from a spore wall). Sources: GOC:lr Also known as: spore germination on or near host Relationships: is a type of GO:0048869 Subtypes: encysted zoospore germination [GO:0075226], conidium germination [GO:0120164] Regulation: regulated by GO:1904359; negatively regulated by negative regulation of spore germination [GO:1904360]; positively regulated by positive regulation of spore germination [GO:1904361]